{
  "term_label": "extracellular matrix organization",
  "term_id": "GO:0030198",
  "gene_name": "Matrix metalloproteinase-15",
  "gene": "UniProtKB:P51511",
  "gene_symbol": "MMP15"
}